{
  "gene_symbol": "UNC93B1",
  "gene_name": "Protein unc-93 homolog B1",
  "term_label": "toll-like receptor 9 signaling pathway",
  "term_id": "GO:0034162",
  "gene": "UniProtKB:Q9H1C4"
}